{
  "gene": "UniProtKB:Q8TAD4",
  "gene_name": "Proton-coupled zinc antiporter SLC30A5",
  "term_id": "GO:1904257",
  "term_label": "zinc ion import into Golgi lumen",
  "gene_symbol": "SLC30A5"
}